{
  "term_label": "Unknown cellular component",
  "gene": "UniProtKB:Q9H2L5",
  "gene_symbol": "RASSF4",
  "term_id": "UNKNOWN:0003",
  "gene_name": "Ras association domain-containing protein 4"
}